{
  "gene": "UniProtKB:Q96ME1",
  "gene_symbol": "FBXL18",
  "gene_name": "F-box_LRR-repeat protein 18",
  "term_label": "Unknown biological process",
  "term_id": "UNKNOWN:0002"
}